{
  "term_label": "plasma membrane",
  "gene_name": "Carcinoembryonic antigen-related cell adhesion molecule 5",
  "term_id": "GO:0005886",
  "gene_symbol": "CEACAM5",
  "gene": "UniProtKB:P06731"
}